S-methylmethionine cycle [GO:0033528] (biological process) Definition: A cyclic series of interconversions involving S-methyl-L-methionine, S-adenosyl-L-homocysteine, S-adenosyl-L-methionine, L-homocysteine, and L-methionine. Converts the methionine group of adenosylmethionine back to free methionine, and may serve regulate the cellular adenosylmethionine level. Relationships: is a type of S-methylmethionine metabolic process [GO:0033477] Sources: GOC:mah, MetaCyc:PWY-5441